T=2 icosahedral viral capsid [GO:0039616] (cellular component) Note: The T=2 symmetry is an non-official appellation; strictly speaking the capsid has a T=1 symmetry with each unit composed of a homodimer. Definition: The protein coat that surrounds the infective nucleic acid in some virus particles where the subunits (capsomeres) are arranged to form an icosahedron with T=2 symmetry. The T=2 capsid is composed of 12 pentameric dimers. Sources: VZ:838 Relationships: is a type of icosahedral viral capsid [GO:0019030]